{
  "gene_symbol": "AXIN2",
  "gene": "UniProtKB:Q9Y2T1",
  "term_id": "GO:0090090",
  "term_label": "negative regulation of canonical Wnt signaling pathway",
  "gene_name": "Axin-2"
}